regulation of interleukin-16 production [GO:0032659] (biological process) Subtypes: negative regulation of interleukin-16 production [GO:0032699], positive regulation of interleukin-16 production [GO:0032739] Also known as: regulation of IL-16 production, regulation of interleukin-16 biosynthetic process Definition: Any process that modulates the frequency, rate, or extent of interleukin-16 production. Sources: GOC:mah Relationships: is a type of regulation of cytokine production [GO:0001817]; regulates interleukin-16 production [GO:0032619]